{
  "term_id": "GO:0004020",
  "gene_name": "Bifunctional 3'-phosphoadenosine 5'-phosphosulfate synthase 1",
  "term_label": "adenylylsulfate kinase activity",
  "gene": "UniProtKB:O43252",
  "gene_symbol": "PAPSS1"
}